{
  "gene_symbol": "SLC5A1",
  "term_id": "GO:0005412",
  "gene": "UniProtKB:P13866",
  "gene_name": "Sodium_glucose cotransporter 1",
  "term_label": "D-glucose:sodium symporter activity"
}